{
  "term_id": "UNKNOWN:0003",
  "gene": "UniProtKB:Q9NWX5",
  "gene_symbol": "ASB6",
  "gene_name": "Ankyrin repeat and SOCS box protein 6",
  "term_label": "Unknown cellular component"
}